{
  "gene_symbol": "LST1",
  "gene": "UniProtKB:O00453",
  "term_label": "Unknown molecular function",
  "gene_name": "Leukocyte-specific transcript 1 protein",
  "term_id": "UNKNOWN:0001"
}